{
  "gene": "UniProtKB:O95935",
  "term_label": "regulation of transcription by RNA polymerase II",
  "term_id": "GO:0006357",
  "gene_symbol": "TBX18",
  "gene_name": "T-box transcription factor TBX18"
}